{
  "term_label": "beta-catenin binding",
  "gene_name": "Vinculin",
  "gene_symbol": "VCL",
  "term_id": "GO:0008013",
  "gene": "UniProtKB:P18206"
}